{
  "term_id": "GO:0022008",
  "gene_name": "Huntingtin-associated protein 1",
  "term_label": "neurogenesis",
  "gene": "UniProtKB:P54257",
  "gene_symbol": "HAP1"
}